{
  "gene_name": "Serum amyloid A-4 protein",
  "term_id": "UNKNOWN:0001",
  "term_label": "Unknown molecular function",
  "gene": "UniProtKB:P35542",
  "gene_symbol": "SAA4"
}